{
  "gene_name": "Interleukin-8",
  "gene_symbol": "CXCL8",
  "term_label": "antimicrobial humoral immune response mediated by antimicrobial peptide",
  "term_id": "GO:0061844",
  "gene": "UniProtKB:P10145"
}